{
  "gene_symbol": "AGAP2",
  "gene_name": "Arf-GAP with GTPase, ANK repeat and PH domain-containing protein 2",
  "gene": "UniProtKB:Q99490",
  "term_id": "GO:0005096",
  "term_label": "GTPase activator activity"
}